{
  "gene_symbol": "RPP40",
  "term_label": "ribonuclease P activity",
  "gene": "UniProtKB:O75818",
  "gene_name": "Ribonuclease P protein subunit p40",
  "term_id": "GO:0004526"
}